{
  "term_id": "UNKNOWN:0002",
  "term_label": "Unknown biological process",
  "gene_name": "Origin recognition complex subunit 2",
  "gene_symbol": "ORC2",
  "gene": "UniProtKB:Q13416"
}